{
  "gene_symbol": "CYP27A1",
  "term_id": "GO:0036378",
  "gene": "UniProtKB:Q02318",
  "gene_name": "Sterol 26-hydroxylase, mitochondrial",
  "term_label": "calcitriol biosynthetic process from calciol"
}